sepal vascular tissue pattern formation [GO:0080057] (biological process) References: PMID:17369435 Definition: Vascular tissue pattern formation as it occurs in the sepal of vascular plants. Relationships: is_a xylem and phloem pattern formation [GO:0010051]